{
  "term_label": "cytosol",
  "gene_symbol": "ADH6",
  "term_id": "GO:0005829",
  "gene": "UniProtKB:P28332",
  "gene_name": "Alcohol dehydrogenase 6"
}